{
  "term_label": "RNA helicase activity",
  "gene_symbol": "DHX9",
  "term_id": "GO:0003724",
  "gene": "UniProtKB:Q08211",
  "gene_name": "ATP-dependent RNA helicase A"
}